non-recombinational interstrand cross-link repair [GO:0036299] (biological process) Relationships: is a type of interstrand cross-link repair [GO:0036297] Definition: Removal of a DNA interstrand crosslink (a covalent attachment of DNA bases on opposite strands of the DNA) and restoration of the DNA by a mechanism that does not involve homologous DNA recombination. References: PMID:11154259, PMID:22064477 Sources: GOC:vw Also known as: recombination-independent ICL repair, recombination-independent interstrand cross-link repair